{
  "gene_name": "Mas-related G-protein coupled receptor member E",
  "gene_symbol": "MRGPRE",
  "term_id": "GO:0007186",
  "term_label": "G protein-coupled receptor signaling pathway",
  "gene": "UniProtKB:Q86SM8"
}